{
  "gene_name": "Vacuolar protein sorting-associated protein 4B",
  "term_id": "GO:0043162",
  "term_label": "ubiquitin-dependent protein catabolic process via the multivesicular body sorting pathway",
  "gene_symbol": "VPS4B",
  "gene": "UniProtKB:O75351"
}